{
  "gene": "UniProtKB:Q8IVV2",
  "term_label": "stereocilium",
  "gene_symbol": "LOXHD1",
  "term_id": "GO:0032420",
  "gene_name": "Lipoxygenase homology domain-containing protein 1"
}